{
  "gene_symbol": "TNFSF14",
  "term_id": "GO:2001238",
  "gene_name": "Tumor necrosis factor ligand superfamily member 14",
  "term_label": "positive regulation of extrinsic apoptotic signaling pathway",
  "gene": "UniProtKB:O43557"
}